{
  "term_label": "Unknown molecular function",
  "gene": "UniProtKB:Q5T4B2",
  "gene_name": "Inactive glycosyltransferase 25 family member 3",
  "gene_symbol": "CERCAM",
  "term_id": "UNKNOWN:0001"
}